8-hydroxygeraniol dehydrogenase activity [GO:0102311] (molecular function) Definition: Catalysis of the reaction: (6E)-8-hydroxygeraniol + 2 NADP = (6E)-8-oxogeranial + 2 NADPH + 2 H+. Sources: EC:1.1.1.324, GOC:pz Relationships: is a type of oxidoreductase activity, acting on the CH-OH group of donors, NAD or NADP as acceptor [GO:0016616]